{
  "gene": "UniProtKB:Q9UJU6",
  "gene_symbol": "DBNL",
  "term_id": "GO:0006897",
  "term_label": "endocytosis",
  "gene_name": "Drebrin-like protein"
}